imaginal disc morphogenesis [GO:0007560] (biological process) Relationships: is a type of animal organ morphogenesis [GO:0009887]; is part of GO:0007444; is part of metamorphosis [GO:0007552]; is part of instar larval or pupal morphogenesis [GO:0048707] Sources: GOC:jid Definition: The process in which the anatomical structures derived from an imaginal disc are generated and organized. The imaginal discs are epithelial infoldings in the larvae of holometabolous insects that develop into adult appendages (legs, antennae, wings, etc.) during metamorphosis from larval to adult form. Also known as: imaginal disc metamorphosis Subtypes: clypeo-labral disc morphogenesis [GO:0007453], labial disc morphogenesis [GO:0007454], eye-antennal disc morphogenesis [GO:0007455], prothoracic disc morphogenesis [GO:0007470], wing disc morphogenesis [GO:0007472], GO:0007478, haltere disc morphogenesis [GO:0007481], genital disc morphogenesis [GO:0007483], histoblast morphogenesis [GO:0007488]